{
  "gene_symbol": "THUMPD1",
  "term_label": "tRNA modification",
  "gene_name": "THUMP domain-containing protein 1",
  "term_id": "GO:0006400",
  "gene": "UniProtKB:Q9NXG2"
}